GPI-linked ephrin receptor activity [GO:0005004] (molecular function) Definition: Combining with a GPI-anchored ephrin to initiate a change in cell activity. References: PMID:9530499 Sources: GOC:mah Also known as: GPI-linked Eph receptor activity Relationships: is a type of ephrin receptor activity [GO:0005003]